{
  "term_label": "Unknown molecular function",
  "gene_symbol": "KRTAP4-3",
  "gene_name": "Keratin-associated protein 4-3",
  "gene": "UniProtKB:Q9BYR4",
  "term_id": "UNKNOWN:0001"
}